positive regulation of VCP-NPL4-UFD1 AAA ATPase complex assembly [GO:1904241] (biological process) Sources: GOC:PARL, GOC:TermGenie, GOC:bf, GO_REF:0000058 Definition: Any process that activates or increases the frequency, rate or extent of VCP-NPL4-UFD1 AAA ATPase complex assembly. Relationships: is a type of positive regulation of protein-containing complex assembly [GO:0031334]; is a type of regulation of VCP-NPL4-UFD1 AAA ATPase complex assembly [GO:1904239]; positively regulates VCP-NPL4-UFD1 AAA ATPase complex assembly [GO:1904210] Also known as: positive regulation of VCP-NPL4-UFD1 AAA ATPase complex formation, positive regulation of p97-Ufd1-Npl4 complex assembly, positive regulation of p97-Ufd1-Npl4 complex formation, up regulation of VCP-NPL4-UFD1 AAA ATPase complex assembly, up regulation of VCP-NPL4-UFD1 AAA ATPase complex formation, up regulation of p97-Ufd1-Npl4 complex assembly, up regulation of p97-Ufd1-Npl4 complex formation, up-regulation of VCP-NPL4-UFD1 AAA ATPase complex assembly, up-regulation of VCP-NPL4-UFD1 AAA ATPase complex formation, up-regulation of p97-Ufd1-Npl4 complex assembly, up-regulation of p97-Ufd1-Npl4 complex formation, upregulation of VCP-NPL4-UFD1 AAA ATPase complex assembly, upregulation of VCP-NPL4-UFD1 AAA ATPase complex formation, upregulation of p97-Ufd1-Npl4 complex assembly, upregulation of p97-Ufd1-Npl4 complex formation, activation of Cdc48p-Npl4p-Ufd1p AAA ATPase complex assembly, activation of Cdc48p-Npl4p-Ufd1p AAA ATPase complex formation, activation of VCP-NPL4-UFD1 AAA ATPase complex assembly, activation of VCP-NPL4-UFD1 AAA ATPase complex formation, activation of p97-Ufd1-Npl4 complex assembly, activation of p97-Ufd1-Npl4 complex formation, positive regulation of Cdc48p-Npl4p-Ufd1p AAA ATPase complex assembly, positive regulation of Cdc48p-Npl4p-Ufd1p AAA ATPase complex formation, up regulation of Cdc48p-Npl4p-Ufd1p AAA ATPase complex assembly, up regulation of Cdc48p-Npl4p-Ufd1p AAA ATPase complex formation, up-regulation of Cdc48p-Npl4p-Ufd1p AAA ATPase complex assembly, up-regulation of Cdc48p-Npl4p-Ufd1p AAA ATPase complex formation, upregulation of Cdc48p-Npl4p-Ufd1p AAA ATPase complex assembly, upregulation of Cdc48p-Npl4p-Ufd1p AAA ATPase complex formation